{
  "gene_name": "RNA-binding motif protein, Y chromosome, family 1 member A1",
  "gene_symbol": "RBMY1A1",
  "term_id": "GO:0003729",
  "gene": "UniProtKB:P0DJD3",
  "term_label": "mRNA binding"
}